{
  "gene_symbol": "TP53I11",
  "gene_name": "Tumor protein p53-inducible protein 11",
  "term_id": "UNKNOWN:0002",
  "term_label": "Unknown biological process",
  "gene": "UniProtKB:O14683"
}